interleukin-12-interleukin-12 receptor complex [GO:0070023] (cellular component) Also known as: IL12-IL12 receptor complex, IL12B-IL12RB1-IL12RB2 complex Definition: A protein complex that is formed by the association of a heterodimeric interleukin-12 receptor complex with an interleukin-12 heterodimer. Relationships: is a type of plasma membrane protein complex [GO:0098797] References: PMID:11900991